{
  "gene_symbol": "WWC1",
  "gene": "UniProtKB:Q8IX03",
  "term_id": "GO:0046621",
  "term_label": "negative regulation of organ growth",
  "gene_name": "Protein KIBRA"
}